{
  "term_label": "receptor ligand activity",
  "gene": "UniProtKB:Q7Z5A8",
  "gene_name": "Chemokine-like protein TAFA-3",
  "gene_symbol": "TAFA3",
  "term_id": "GO:0048018"
}